farnesol metabolic process [GO:0016487] (biological process) Relationships: is a type of sesquiterpenoid metabolic process [GO:0006714]; is a type of polyprenol metabolic process [GO:0016093]; is a type of primary alcohol metabolic process [GO:0034308] Definition: The chemical reactions and pathways involving the sesquiterpenoid alcohol farnesol, 3,7,11-trimethyl-2,6,10,dodecatrien-1-ol. Sources: GOC:go_curators Also known as: farnesol metabolism Subtypes: farnesol biosynthetic process [GO:0006715], GO:0016488